{
  "term_label": "piRNA processing",
  "gene_symbol": "HENMT1",
  "term_id": "GO:0034587",
  "gene_name": "Small RNA 2'-O-methyltransferase",
  "gene": "UniProtKB:Q5T8I9"
}